{
  "term_label": "plasma membrane",
  "gene_symbol": "GAS1",
  "term_id": "GO:0005886",
  "gene_name": "Growth arrest-specific protein 1",
  "gene": "UniProtKB:P54826"
}